{
  "gene_name": "Protein AF1q",
  "term_id": "GO:0005654",
  "gene": "UniProtKB:Q13015",
  "term_label": "nucleoplasm",
  "gene_symbol": "MLLT11"
}